{
  "term_id": "GO:0005739",
  "term_label": "mitochondrion",
  "gene_symbol": "MCAT",
  "gene": "UniProtKB:Q8IVS2",
  "gene_name": "Malonyl-CoA-acyl carrier protein transacylase, mitochondrial"
}